positive regulation of receptor-mediated virion attachment to host cell [GO:1902736] (biological process) Relationships: is a type of GO:1902734; is a type of GO:1903902; positively regulates receptor-mediated virion attachment to host cell [GO:0046813] Definition: Any process that activates or increases the frequency, rate or extent of receptor-mediated virion attachment to host cell. References: PMID:18385238 Sources: GOC:TermGenie, GOC:als, GO_REF:0000058 Also known as: positive regulation of virion attachment, binding of host cell surface receptor, up regulation of receptor-mediated virion attachment to host cell, up regulation of virion attachment, binding of host cell surface receptor, up-regulation of receptor-mediated virion attachment to host cell, up-regulation of virion attachment, binding of host cell surface receptor, upregulation of receptor-mediated virion attachment to host cell, upregulation of virion attachment, binding of host cell surface receptor, activation of receptor-mediated virion attachment to host cell, activation of virion attachment, binding of host cell surface receptor